{
  "gene_name": "WD repeat and HMG-box DNA-binding protein 1",
  "term_id": "GO:0006281",
  "term_label": "DNA repair",
  "gene_symbol": "WDHD1",
  "gene": "UniProtKB:O75717"
}